{
  "term_label": "minus-end-directed microtubule motor activity",
  "gene_symbol": "DNAH5",
  "gene": "UniProtKB:Q8TE73",
  "term_id": "GO:0008569",
  "gene_name": "Dynein axonemal heavy chain 5"
}